{
  "gene": "UniProtKB:Q6ZMH5",
  "gene_symbol": "SLC39A5",
  "gene_name": "Zinc transporter ZIP5",
  "term_label": "zinc ion import across plasma membrane",
  "term_id": "GO:0071578"
}